{
  "gene_symbol": "MRPL4",
  "term_label": "structural constituent of ribosome",
  "gene": "UniProtKB:Q9BYD3",
  "gene_name": "Large ribosomal subunit protein uL4m",
  "term_id": "GO:0003735"
}